antigen processing and presentation of peptide antigen via MHC class I [GO:0002474] (biological process) Subtypes: GO:0019885, antigen processing and presentation of exogenous peptide antigen via MHC class I [GO:0042590] References: PMID:15224092, PMID:15771591 Sources: GOC:add, ISBN:0781735149 Regulation: regulated by regulation of antigen processing and presentation of peptide antigen via MHC class I [GO:0002589]; negatively regulated by GO:0002590; positively regulated by positive regulation of antigen processing and presentation of peptide antigen via MHC class I [GO:0002591] Also known as: peptide antigen processing and presentation via MHC class I Relationships: is a type of antigen processing and presentation of peptide antigen [GO:0048002] Definition: The process in which an antigen-presenting cell expresses a peptide antigen on its cell surface in association with an MHC class I protein complex. Class I here refers to classical class I molecules.